{
  "gene_name": "Lung adenoma susceptibility protein 2",
  "term_label": "Unknown cellular component",
  "gene": "UniProtKB:Q8IYD9",
  "term_id": "UNKNOWN:0003",
  "gene_symbol": "LAS2"
}